{
  "term_id": "GO:0031267",
  "term_label": "small GTPase binding",
  "gene_name": "EH domain-binding protein 1-like protein 1",
  "gene_symbol": "EHBP1L1",
  "gene": "UniProtKB:Q8N3D4"
}